{
  "gene": "UniProtKB:P60520",
  "term_id": "GO:0000045",
  "gene_name": "Gamma-aminobutyric acid receptor-associated protein-like 2",
  "term_label": "autophagosome assembly",
  "gene_symbol": "GABARAPL2"
}